{
  "gene_symbol": "MAPKAPK2",
  "term_label": "response to cytokine",
  "gene": "UniProtKB:P49137",
  "gene_name": "MAP kinase-activated protein kinase 2",
  "term_id": "GO:0034097"
}